inhibitory chemical synaptic transmission [GO:0098977] (biological process) Relationships: is a type of chemical synaptic transmission [GO:0007268]; has part inhibitory postsynaptic potential [GO:0060080] Sources: GOC:dos Definition: Synaptic transmission that results in an inhibitory postsynaptic potential.